zinc ion import into synaptic vesicle [GO:0099180] (biological process) Also known as: Zn2+ import into synaptic vesicle, zinc import into synaptic vesicle Definition: The directed movement of Zn2+ ions from the cytoplasm into the lumen of a cytoplasmic vesicle. References: PMID:9990090 Relationships: is_a GO:0062111